{
  "term_label": "extracellular matrix structural constituent conferring tensile strength",
  "gene_name": "Collagen alpha-1(VIII) chain",
  "term_id": "GO:0030020",
  "gene_symbol": "COL8A1",
  "gene": "UniProtKB:P27658"
}